{
  "gene": "UniProtKB:Q8NG41",
  "gene_name": "Neuropeptide B",
  "gene_symbol": "NPB",
  "term_label": "G protein-coupled receptor binding",
  "term_id": "GO:0001664"
}